{
  "gene_symbol": "RCCD1",
  "gene_name": "RCC1 domain-containing protein 1",
  "gene": "UniProtKB:A6NED2",
  "term_label": "Unknown biological process",
  "term_id": "UNKNOWN:0002"
}